locomotory behavior [GO:0007626] (biological process) Relationships: is a type of behavior [GO:0007610] Sources: GOC:dph Also known as: behavior via locomotion, locomotion in response to stimulus, locomotory behavioral response to stimulus, locomotory behaviour, locomotory behavioural response to stimulus Definition: The specific movement from place to place of an organism in response to external or internal stimuli. Locomotion of a whole organism in a manner dependent upon some combination of that organism's internal state and external conditions. Subtypes: adult locomotory behavior [GO:0008344], larval locomotory behavior [GO:0008345], turning behavior [GO:0035178], locomotory exploration behavior [GO:0035641], swimming behavior [GO:0036269], locomotor rhythm [GO:0045475], walking behavior [GO:0090659]